{
  "gene_name": "Tyrosine-protein kinase Fgr",
  "gene_symbol": "FGR",
  "term_label": "cell surface receptor protein tyrosine kinase signaling pathway",
  "gene": "UniProtKB:P09769",
  "term_id": "GO:0007169"
}